{
  "term_id": "UNKNOWN:0003",
  "gene_symbol": "SPRY3",
  "gene": "UniProtKB:O43610",
  "gene_name": "Protein sprouty homolog 3",
  "term_label": "Unknown cellular component"
}